postsynaptic density assembly [GO:0097107] (biological process) Also known as: PSD assembly, post synaptic density assembly, post-synaptic density assembly Relationships: is a type of GO:0097106; is a type of postsynaptic specialization assembly [GO:0098698]; is part of excitatory synapse assembly [GO:1904861] Definition: The aggregation, arrangement and bonding together of a set of components to form a postsynaptic density, a region that lies adjacent to the cytoplasmic face of the postsynaptic membrane at excitatory synapse. Regulation: regulated by regulation of postsynaptic density assembly [GO:0099151]; positively regulated by GO:0160036; negatively regulated by negative regulation of postsynaptic density assembly [GO:0160037] References: PMID:21525273 Sources: GOC:BHF, GOC:sjp